mannan polymerase I complex [GO:0140498] (CC) Definition: A complex with alpha-(1->6)-mannosyltransferase activity, located in the cis Golgi membrane; adds mannan to N-linked glycans on proteins as part of the priming and elongation of alpha 1,6-linked Man backbone. In S. cerevisiae, contains Mnn9p and Van1p. Relationships: is a type of mannan polymerase complex [GO:0000136] References: PMID:9430634